{
  "gene_symbol": "TYROBP",
  "gene": "UniProtKB:O43914",
  "term_id": "GO:0002282",
  "gene_name": "TYRO protein tyrosine kinase-binding protein",
  "term_label": "microglial cell activation involved in immune response"
}